{
  "term_id": "UNKNOWN:0001",
  "gene_name": "Enoyl-CoA hydratase, mitochondrial",
  "gene_symbol": "ECHS1",
  "gene": "UniProtKB:P30084",
  "term_label": "Unknown molecular function"
}